{
  "term_label": "intrinsic apoptotic signaling pathway in response to DNA damage",
  "gene_symbol": "BCL2",
  "term_id": "GO:0008630",
  "gene_name": "Apoptosis regulator Bcl-2",
  "gene": "UniProtKB:P10415"
}